adenylate cyclase-activating dopamine receptor signaling pathway [GO:0007191] (biological process) Also known as: dopamine receptor, adenylate cyclase activating pathway, dopamine receptor, adenylyl cyclase activating pathway, activation of adenylate cyclase activity by dopamine receptor signaling pathway, activation of adenylate cyclase activity by dopamine receptor signalling pathway Sources: GOC:mah, GOC:signaling Definition: An adenylate cyclase-activating G protein-coupled receptor signaling pathway initiated by dopamine binding to its receptor, and ending with the regulation of a downstream cellular process. Relationships: is a type of adenylate cyclase-activating G protein-coupled receptor signaling pathway [GO:0007189]; is_a G protein-coupled dopamine receptor signaling pathway [GO:0007212]